{
  "gene_symbol": "ZDHHC18",
  "gene_name": "Palmitoyltransferase ZDHHC18",
  "term_label": "Golgi apparatus",
  "term_id": "GO:0005794",
  "gene": "UniProtKB:Q9NUE0"
}